{
  "gene_name": "Epoxide hydrolase 1",
  "gene_symbol": "EPHX1",
  "gene": "UniProtKB:P07099",
  "term_id": "GO:0019369",
  "term_label": "arachidonate metabolic process"
}